cellular bud neck polarisome [GO:0031560] (cellular component) Definition: Protein complex that has a role in determining cell polarity, found at the neck of a fungal bud before and during cytokinesis. References: PMID:9632790 Relationships: is a type of polarisome [GO:0000133]; is part of cellular bud neck [GO:0005935]